HMG box domain binding [GO:0071837] (molecular function) Relationships: is a type of protein domain specific binding [GO:0019904] Definition: Binding to an HMG box domain, a protein domain that consists of three helices in an irregular array. HMG-box domains are found in one or more copies in HMG-box proteins, which form a large, diverse family involved in the regulation of DNA-dependent processes such as transcription, replication, and strand repair, all of which require the bending and unwinding of chromatin. References: PMID:18445004 Sources: GOC:yaf, InterPro:IPR009071